{
  "gene_name": "Protein YIPF4",
  "term_id": "GO:0006888",
  "term_label": "endoplasmic reticulum to Golgi vesicle-mediated transport",
  "gene": "UniProtKB:Q9BSR8",
  "gene_symbol": "YIPF4"
}